{
  "gene": "UniProtKB:Q9H7Z6",
  "term_label": "Unknown biological process",
  "gene_symbol": "KAT8",
  "gene_name": "Histone acetyltransferase KAT8",
  "term_id": "UNKNOWN:0002"
}